{
  "gene_name": "Collagen alpha-1(VI) chain",
  "gene": "UniProtKB:P12109",
  "gene_symbol": "COL6A1",
  "term_label": "Unknown molecular function",
  "term_id": "UNKNOWN:0001"
}